{
  "gene_symbol": "GRIK5",
  "gene_name": "Glutamate receptor ionotropic, kainate 5",
  "term_label": "postsynaptic density membrane",
  "gene": "UniProtKB:Q16478",
  "term_id": "GO:0098839"
}